lipoxin A4 metabolic process [GO:2001302] (BP) Also known as: LXA4 metabolic process, LXA4 metabolism, lipoxin A4 metabolism Definition: The chemical reactions and pathways involving lipoxin A4. Lipoxin A4 is a C20 hydroxy fatty acid having (5S)-, (6R)- and (15S)-hydroxy groups as well as (7E)- (9E)-, (11Z)- and (13E)-double bonds. Sources: GOC:mw Subtypes: lipoxin A4 biosynthetic process [GO:2001303] Relationships: is a type of long-chain fatty acid metabolic process [GO:0001676]; is a type of unsaturated fatty acid metabolic process [GO:0033559]; is a type of fatty acid derivative metabolic process [GO:1901568]